plasma lipoprotein particle disassembly [GO:0071829] (biological process) Relationships: is a type of protein-lipid complex disassembly [GO:0032987]; is a type of plasma lipoprotein particle organization [GO:0071827]; is part of regulation of plasma lipoprotein particle levels [GO:0097006] Sources: GOC:mah Subtypes: low-density lipoprotein particle disassembly [GO:0090495] Definition: The disaggregation of a plasma lipoprotein particle into its constituent components.